skin morphogenesis [GO:0043589] (biological process) Relationships: is a type of animal organ morphogenesis [GO:0009887]; is part of skin development [GO:0043588] Sources: GOC:jl, UBERON:0002097 Definition: The process in which the anatomical structures of the skin are generated and organized. The skin is the external membranous integument of an animal. In vertebrates the skin generally consists of two layers, an outer nonsensitive and nonvascular epidermis (cuticle or skarfskin) composed of cells which are constantly growing and multiplying in the deeper, and being thrown off in the superficial layers, as well as an inner, sensitive and vascular dermis (cutis, corium or true skin) composed mostly of connective tissue.